{
  "term_label": "Unknown molecular function",
  "gene_name": "Nucleolar and coiled-body phosphoprotein 1",
  "term_id": "UNKNOWN:0001",
  "gene_symbol": "NOLC1",
  "gene": "UniProtKB:Q14978"
}